{
  "gene_name": "Uncharacterized protein C9orf57",
  "term_label": "Unknown molecular function",
  "gene": "UniProtKB:Q5W0N0",
  "gene_symbol": "C9orf57",
  "term_id": "UNKNOWN:0001"
}